oxoadipate dehydrogenase complex [GO:0160167] (CC) Definition: A multi-enzyme complex that catalyzes the oxidative decarboxylation of 2-oxoadipate to glutaryl-CoA, thereby acting in the final step of lysine and tryptophan catabolism in mitochondria. The complex comprises multiple copies of three enzymes referred to as E1, E2 and E3: 2-oxoadipate dehydrogenase (E1), dihydrolipoamide S-succinyltransferase (E2) and dihydrolipoamide dehydrogenase (E3). Relationships: is a type of GO:0045240 References: PMID:29191460, PMID:32695416 Also known as: OADHC Note: The catalytic activities of the individual components of this complex are represented by the molecular function terms '2-oxoadipate dehydrogenase activity ; GO:0160166' (E1), 'dihydrolipoyllysine-residue succinyltransferase activity ; GO:0004149' (E2), and 'dihydrolipoyl dehydrogenase activity ; GO:0004148' (E3).